{
  "term_id": "GO:0005615",
  "term_label": "extracellular space",
  "gene_name": "Pro-neuregulin-3, membrane-bound isoform",
  "gene": "UniProtKB:P56975",
  "gene_symbol": "NRG3"
}